regulation of RNA import into nucleus [GO:0046828] (biological process) Relationships: is a type of GO:0032239; is a type of GO:0046822; regulates RNA import into nucleus [GO:0006404] Also known as: regulation of RNA import into cell nucleus, regulation of RNA transport from cytoplasm to nucleus, regulation of RNA-nucleus import Sources: GOC:bf Subtypes: negative regulation of RNA import into nucleus [GO:0046829], positive regulation of RNA import into nucleus [GO:0046830] Definition: Any process that modulates the frequency, rate or extent of movement of RNA from the cytoplasm to the nucleus.